{
  "gene": "UniProtKB:Q9NTM9",
  "term_label": "copper ion binding",
  "gene_symbol": "CUTC",
  "term_id": "GO:0005507",
  "gene_name": "Copper homeostasis protein cutC homolog"
}